glyceraldehyde-3-phosphate dehydrogenase (NADP+) (phosphorylating) activity [GO:0047100] (molecular function) Sources: EC:1.2.1.13, MetaCyc:1.2.1.13-RXN Relationships: is a type of GO:0043891 Definition: Catalysis of the reaction: phosphate + NADP+ + glyceraldehyde-3-phosphate = NADPH + 3-phospho-D-glyceroyl-phosphate. Also known as: D-glyceraldehyde-3-phosphate:NADP+ oxidoreductase (phosphorylating), NADP-dependent glyceraldehyde phosphate dehydrogenase activity, NADP-dependent glyceraldehyde-3-phosphate dehydrogenase activity, NADP-triose phosphate dehydrogenase activity, dehydrogenase, glyceraldehyde phosphate (nicotinamide adenine dinucleotide phosphate) (phosphorylating), glyceraldehyde phosphate dehydrogenase (nicotinamide adenine dinucleotide phosphate) (phosphorylating), triosephosphate dehydrogenase (NADP(+)) activity, triosephosphate dehydrogenase (NADP), triosephosphate dehydrogenase (NADP+) activity